anthocyanidin 3-glucoside rhamnosyltransferase activity [GO:0051566] (MF) References: PMID:8130800 Also known as: 3RT activity, anthocyanidin 3-glucoside-rhamnosyltransferase activity Definition: Catalysis of the reaction: anthocyanidin 3-glucoside + UDP-rhamnose = anthocyanidin 3-rutinoside + UDP. Relationships: is a type of hexosyltransferase activity [GO:0016758]